{
  "gene_name": "Tight junction protein ZO-3",
  "gene": "UniProtKB:O95049",
  "term_label": "cell-cell junction organization",
  "gene_symbol": "TJP3",
  "term_id": "GO:0045216"
}